regulation of aerobic respiration [GO:1903715] (biological process) References: PMID:19266076 Sources: GOC:TermGenie, GO_REF:0000058 Subtypes: regulation of oxidative phosphorylation [GO:0002082], GO:1902956 Relationships: is a type of regulation of cellular respiration [GO:0043457]; regulates aerobic respiration [GO:0009060] Definition: Any process that modulates the frequency, rate or extent of aerobic respiration.